{
  "term_id": "UNKNOWN:0002",
  "gene_symbol": "MGAM2",
  "gene_name": "Probable maltase-glucoamylase 2",
  "term_label": "Unknown biological process",
  "gene": "UniProtKB:Q2M2H8"
}